glycerophosphodiester transmembrane transport [GO:0001407] (biological process) Definition: The process in which a glycerophosphodiester is transported across a membrane. Glycerophosphodiesters are small molecules composed of glycerol-3-phosphate and an alcohol, for example, glycerophosphoinositol. Relationships: is a type of GO:0015711; is a type of organophosphate ester transport [GO:0015748]; is a type of transmembrane transport [GO:0055085] References: PMID:12912892 Sources: GOC:mcc